{
  "term_label": "lens development in camera-type eye",
  "gene": "UniProtKB:P53673",
  "term_id": "GO:0002088",
  "gene_symbol": "CRYBA4",
  "gene_name": "Beta-crystallin A4"
}